{
  "term_label": "nucleus",
  "gene": "UniProtKB:Q99941",
  "gene_symbol": "ATF6B",
  "term_id": "GO:0005634",
  "gene_name": "Cyclic AMP-dependent transcription factor ATF-6 beta"
}